taxis [GO:0042330] (biological process) Definition: The directed movement of a motile cell or organism in response to an external stimulus. Sources: GOC:jl, ISBN:0192801023 Subtypes: chemotaxis [GO:0006935], energy taxis [GO:0009453], interneuron sorting involved in substrate-independent cerebral cortex tangential migration [GO:0021844], gravitaxis [GO:0042332], thermotaxis [GO:0043052] Also known as: directed movement in response to stimulus Relationships: is a type of locomotion [GO:0040011]; is part of response to external stimulus [GO:0009605]